{
  "term_label": "mRNA binding",
  "term_id": "GO:0003729",
  "gene_symbol": "RBMXL3",
  "gene_name": "RNA-binding motif protein, X-linked-like-3",
  "gene": "UniProtKB:Q8N7X1"
}